{
  "gene_name": "Carbohydrate sulfotransferase 9",
  "term_id": "GO:0030166",
  "term_label": "proteoglycan biosynthetic process",
  "gene_symbol": "CHST9",
  "gene": "UniProtKB:Q7L1S5"
}